{
  "term_label": "Unknown biological process",
  "gene_name": "RNA-binding protein MEX3B",
  "gene_symbol": "MEX3B",
  "term_id": "UNKNOWN:0002",
  "gene": "UniProtKB:Q6ZN04"
}